proepicardium cell migration involved in pericardium morphogenesis [GO:0003345] (biological process) Relationships: is a type of cell migration involved in heart development [GO:0060973]; is part of pericardium morphogenesis [GO:0003344] References: PMID:18722343 Sources: GOC:dph Definition: The coordinated movement of a mesenchymal proepicardial cell to the surface of the developing heart.